{
  "gene": "UniProtKB:A6NF89",
  "term_label": "Unknown biological process",
  "gene_name": "Olfactory receptor 6C6",
  "gene_symbol": "OR6C6",
  "term_id": "UNKNOWN:0002"
}